{
  "term_id": "GO:0005179",
  "gene_symbol": "CSH2",
  "gene_name": "Chorionic somatomammotropin hormone 2",
  "term_label": "hormone activity",
  "gene": "UniProtKB:P0DML3"
}